{
  "term_id": "GO:0008422",
  "gene_symbol": "GBA2",
  "gene": "UniProtKB:Q9HCG7",
  "term_label": "beta-glucosidase activity",
  "gene_name": "Non-lysosomal glucosylceramidase"
}